{
  "gene": "UniProtKB:Q96EL2",
  "term_id": "UNKNOWN:0003",
  "term_label": "Unknown cellular component",
  "gene_symbol": "MRPS24",
  "gene_name": "Small ribosomal subunit protein uS3m"
}